rhombomere 1 structural organization [GO:0021653] (biological process) Relationships: is a type of rhombomere structural organization [GO:0021595]; is part of GO:0021651 Definition: The process that contributes to creating the structural organization of rhombomere 1. This process pertains to the physical shaping of a rudimentary structure. Rhombomeres are transverse segments of the developing rhombencephalon. Rhombomeres are lineage restricted, express different genes from one another, and adopt different developmental fates. Rhombomeres are numbered in an anterior to posterior order. Also known as: rhombomere 1 structural organisation Sources: GOC:cls, GOC:dgh, GOC:dph, GOC:jid, GO_REF:0000021